8-amino-7-oxononanoate synthase activity [GO:0008710] (molecular function) Relationships: is_a acyltransferase activity, transferring groups other than amino-acyl groups [GO:0016747] Also known as: 6-carboxyhexanoyl-CoA:L-alanine C-carboxyhexanoyltransferase (decarboxylating), 7-KAP synthetase activity, 7-keto-8-amino-pelargonic acid synthetase activity, 7-keto-8-aminopelargonic acid synthetase activity, 7-keto-8-aminopelargonic synthetase activity, 8-amino-7-ketopelargonate synthase activity, 8-amino-7-oxopelargonate synthase activity, AONS activity Definition: Catalysis of the reaction: L-alanine + H+ + pimelyl-CoA = 8-amino-7-oxononanoate + CO2 + CoA. Sources: EC:2.3.1.47, RHEA:20712